{
  "gene_name": "Membrane-associated guanylate kinase, WW and PDZ domain-containing protein 2",
  "term_id": "GO:0007165",
  "term_label": "signal transduction",
  "gene_symbol": "MAGI2",
  "gene": "UniProtKB:Q86UL8"
}